{
  "term_label": "NMDA glutamate receptor activity",
  "gene_name": "Glutamate receptor ionotropic, NMDA 2D",
  "gene_symbol": "GRIN2D",
  "gene": "UniProtKB:O15399",
  "term_id": "GO:0004972"
}